4-hydroxy-3-all-trans-polyprenylbenzoate oxygenase activity [GO:0106364] (molecular function) Relationships: is a type of oxidoreductase activity, acting on paired donors, with incorporation or reduction of molecular oxygen, reduced iron-sulfur protein as one donor, and incorporation of one atom of oxygen [GO:0016713] References: PMID:38425362 Sources: RHEA:81195 Also known as: 4-hydroxy-3-all-trans-hexaprenylbenzoate oxygenase activity Definition: Catalysis of the reaction: 4-hydroxy-3-all-trans-polyprenylbenzoate + 2 H+ + O2 + 2 reduced [2Fe-2S]-[ferredoxin] = 3,4-dihydroxy-5-all-trans-polyprenylbenzoate + H2O + 2 oxidized [2Fe-2S]-[ferredoxin].